{
  "term_label": "protein tyrosine kinase binding",
  "gene_symbol": "CEACAM7",
  "term_id": "GO:1990782",
  "gene_name": "Carcinoembryonic antigen-related cell adhesion molecule 7",
  "gene": "UniProtKB:Q14002"
}